{
  "term_id": "UNKNOWN:0002",
  "term_label": "Unknown biological process",
  "gene_name": "Uncharacterized protein C2orf72",
  "gene_symbol": "C2orf72",
  "gene": "UniProtKB:A6NCS6"
}